{
  "gene_symbol": "RPS27",
  "gene": "UniProtKB:P42677",
  "gene_name": "Small ribosomal subunit protein eS27",
  "term_label": "RNA binding",
  "term_id": "GO:0003723"
}